{
  "term_label": "Unknown biological process",
  "gene_symbol": "SUGP2",
  "gene": "UniProtKB:Q8IX01",
  "gene_name": "SURP and G-patch domain-containing protein 2",
  "term_id": "UNKNOWN:0002"
}